protein lysine delactylase activity [GO:0160216] (molecular function) Relationships: is a type of GO:0140096; is a type of deacylase activity [GO:0160215] References: PMID:35044827 Sources: RHEA:81387 Definition: Catalysis of the reaction: H2O + N6-lactoyl-L-lysyl-[protein] = (S)-lactate + L-lysyl-[protein].